{
  "gene_symbol": "CD83",
  "term_label": "Unknown biological process",
  "gene_name": "CD83 antigen",
  "term_id": "UNKNOWN:0002",
  "gene": "UniProtKB:Q01151"
}